{
  "term_label": "thiamine diphosphokinase activity",
  "gene_name": "Thiamin pyrophosphokinase 1",
  "gene": "UniProtKB:Q9H3S4",
  "term_id": "GO:0004788",
  "gene_symbol": "TPK1"
}